{
  "term_label": "L-cysteine transaminase activity",
  "gene_name": "CDGSH iron-sulfur domain-containing protein 1",
  "gene_symbol": "CISD1",
  "gene": "UniProtKB:Q9NZ45",
  "term_id": "GO:0047801"
}